medium-chain fatty acyl-CoA dehydrogenase activity [GO:0070991] (MF) Also known as: MCAD activity Sources: RHEA:14477 Note: While there is not universal consensus on the lengths of short-, medium-, long- and very-long-chain fatty acids, the GO uses the definitions in ChEBI (see CHEBI:26666, CHEBI:59554, CHEBI:15904 and CHEBI:27283). Relationships: is_a acyl-CoA dehydrogenase activity [GO:0003995] Definition: Catalysis of the reaction: a medium-chain 2,3-saturated fatty acyl-CoA + H+ + oxidized [electron-transfer flavoprotein] = a medium-chain trans-(2E)-enoyl-CoA + reduced [electron-transfer flavoprotein]. A medium-chain fatty acid has an aliphatic tail containing 6 to 12 carbons.